{
  "gene_symbol": "SLC25A25",
  "gene_name": "Mitochondrial adenyl nucleotide antiporter SLC25A25",
  "term_id": "GO:0015866",
  "term_label": "ADP transport",
  "gene": "UniProtKB:Q6KCM7"
}